membrane lipid metabolic process [GO:0006643] (biological process) Relationships: is a type of lipid metabolic process [GO:0006629]; occurs in GO:0016020 Sources: GOC:ai Subtypes: glycolipid metabolic process [GO:0006664], sphingolipid metabolic process [GO:0006665], membrane lipid catabolic process [GO:0046466], membrane lipid biosynthetic process [GO:0046467] Regulation: regulated by regulation of membrane lipid metabolic process [GO:1905038] Also known as: membrane lipid metabolism Definition: The chemical reactions and pathways involving membrane lipids, any lipid found in or associated with a biological membrane.